{
  "gene_name": "Dynactin subunit 2",
  "gene_symbol": "DCTN2",
  "term_label": "mitotic spindle organization",
  "term_id": "GO:0007052",
  "gene": "UniProtKB:Q13561"
}